regulation of humoral immune response [GO:0002920] (biological process) Subtypes: regulation of antimicrobial humoral response [GO:0002759], negative regulation of humoral immune response [GO:0002921], GO:0002922, regulation of humoral immune response mediated by circulating immunoglobulin [GO:0002923], regulation of complement activation [GO:0030449] Definition: Any process that modulates the frequency, rate, or extent of a humoral immune response. Relationships: is a type of regulation of immune response [GO:0050776]; regulates humoral immune response [GO:0006959] Sources: GOC:add